barbiturase activity [GO:0047694] (molecular function) Definition: Catalysis of the reaction: barbiturate + H2O = malonate + urea. Also known as: barbiturate amidohydrolase (3-oxo-3-ureidopropanoate-forming) Relationships: is a type of hydrolase activity, acting on carbon-nitrogen (but not peptide) bonds, in cyclic amides [GO:0016812] Sources: EC:3.5.2.1, MetaCyc:BARBITURASE-RXN